{
  "gene_symbol": "ZIC4",
  "term_id": "GO:0007417",
  "term_label": "central nervous system development",
  "gene": "UniProtKB:Q8N9L1",
  "gene_name": "Zinc finger protein ZIC 4"
}